{
  "gene_name": "Caldesmon",
  "gene_symbol": "CALD1",
  "term_id": "GO:0003779",
  "gene": "UniProtKB:Q05682",
  "term_label": "actin binding"
}